{
  "term_label": "Unknown cellular component",
  "gene_symbol": "GSDMC",
  "gene": "UniProtKB:Q9BYG8",
  "gene_name": "Gasdermin-C",
  "term_id": "UNKNOWN:0003"
}